{
  "gene_name": "Reduced folate transporter",
  "gene": "UniProtKB:P41440",
  "term_label": "plasma membrane",
  "gene_symbol": "SLC19A1",
  "term_id": "GO:0005886"
}